{
  "term_id": "GO:0001725",
  "term_label": "stress fiber",
  "gene": "UniProtKB:P24844",
  "gene_name": "Myosin regulatory light polypeptide 9",
  "gene_symbol": "MYL9"
}